{
  "gene_name": "Glycogen synthase kinase-3 beta",
  "gene_symbol": "GSK3B",
  "term_label": "cytosol",
  "term_id": "GO:0005829",
  "gene": "UniProtKB:P49841"
}